positive regulation of female pigmentation [GO:0048091] (biological process) Relationships: is a type of positive regulation of developmental pigmentation [GO:0048087]; is a type of regulation of female pigmentation [GO:0048089]; is a type of positive regulation of developmental process [GO:0051094]; is a type of GO:0051240; is a type of positive regulation of reproductive process [GO:2000243]; positively regulates GO:0048095 Also known as: up regulation of female pigmentation, up-regulation of female pigmentation, upregulation of female pigmentation, activation of female pigmentation, stimulation of female pigmentation Sources: GOC:jid Definition: Any process that activates or increases the frequency, rate or extent of establishment of a pattern of pigment in females.